{
  "gene_symbol": "TMTC2",
  "gene": "UniProtKB:Q8N394",
  "gene_name": "Protein O-mannosyl-transferase TMTC2",
  "term_label": "protein O-linked glycosylation via mannose",
  "term_id": "GO:0035269"
}